glutaconate CoA-transferase activity [GO:0018730] (molecular function) Definition: Catalysis of the reaction: acetyl-CoA + (E)-glutaconate = acetate + glutaconyl-1-CoA. Sources: EC:2.8.3.12 Also known as: acetyl-CoA:(E)-glutaconate CoA-transferase activity Relationships: is a type of CoA-transferase activity [GO:0008410]